{
  "term_label": "nucleus",
  "gene_symbol": "HELLS",
  "term_id": "GO:0005634",
  "gene": "UniProtKB:Q9NRZ9",
  "gene_name": "Lymphoid-specific helicase"
}